{
  "gene": "UniProtKB:Q14586",
  "term_id": "GO:0000976",
  "gene_symbol": "ZNF267",
  "term_label": "transcription cis-regulatory region binding",
  "gene_name": "Zinc finger protein 267"
}